{
  "gene": "UniProtKB:Q9HAD4",
  "gene_symbol": "WDR41",
  "term_label": "Unknown cellular component",
  "gene_name": "WD repeat-containing protein 41",
  "term_id": "UNKNOWN:0003"
}